{
  "gene_symbol": "SPACA7",
  "term_label": "Unknown molecular function",
  "gene": "UniProtKB:Q96KW9",
  "gene_name": "Sperm acrosome-associated protein 7",
  "term_id": "UNKNOWN:0001"
}